{
  "term_id": "GO:0007399",
  "term_label": "nervous system development",
  "gene": "UniProtKB:P36896",
  "gene_symbol": "ACVR1B",
  "gene_name": "Activin receptor type-1B"
}